{
  "term_label": "L-aspartate import across plasma membrane",
  "term_id": "GO:0140009",
  "gene": "UniProtKB:Q15758",
  "gene_symbol": "SLC1A5",
  "gene_name": "Neutral amino acid transporter B(0)"
}